{
  "term_id": "GO:0042254",
  "gene": "UniProtKB:Q13620",
  "gene_name": "Cullin-4B",
  "gene_symbol": "CUL4B",
  "term_label": "ribosome biogenesis"
}